{
  "term_label": "laminin receptor activity",
  "gene_symbol": "BCAM",
  "gene_name": "Basal cell adhesion molecule",
  "gene": "UniProtKB:P50895",
  "term_id": "GO:0005055"
}